sympathetic neuron projection guidance [GO:0097491] (biological process) Also known as: sympathetic neuron process guidance, sympathetic neuron protrusion guidance, sympathetic neuronal cell projection guidance, sympathetic neurite guidance References: PMID:22790009 Sources: GOC:BHF, GOC:rl Relationships: is a type of neuron projection guidance [GO:0097485] Definition: The process in which the migration of a sympathetic neuron projection is directed to a specific target site in response to a combination of attractive and repulsive cues.